{
  "gene_name": "Headcase protein homolog",
  "gene": "UniProtKB:Q9UBI9",
  "term_label": "Unknown molecular function",
  "gene_symbol": "HECA",
  "term_id": "UNKNOWN:0001"
}